jasmonoyl-isoleucine-12-hydroxylase activity [GO:0052694] (MF) Definition: Catalysis of the reaction: jasmonoyl-isoleucine + NADPH + H+ + O2 = 12-hydroxy-jasmonoyl-isoleucine + NADP+ + H2O. Relationships: is a type of monooxygenase activity [GO:0004497] References: PMID:21576464 Sources: MetaCyc:RXN-12421